macrophage colony-stimulating factor receptor activity [GO:0005011] (molecular function) Also known as: M-CSF receptor activity, macrophage colony stimulating factor receptor activity, CSF-1, Fms Sources: GOC:mah, GOC:signaling Definition: Combining with macrophage colony-stimulating factor (M-CSF) receptor ligand and transmitting the signal from one side of the membrane to the other to initiate a change in cell activity by catalysis of the reaction: ATP + a protein-L-tyrosine = ADP + a protein-L-tyrosine phosphate. Relationships: is a type of transmembrane receptor protein tyrosine kinase activity [GO:0004714]; is part of macrophage colony-stimulating factor signaling pathway [GO:0038145]